regulation of tight junction disassembly [GO:1905073] (BP) Definition: Any process that modulates the frequency, rate or extent of tight junction disassembly. References: PMID:18718461 Sources: GOC:BHF, GOC:TermGenie, GOC:rl, GO_REF:0000058 Also known as: regulation of occluding cell junction disassembly, regulation of occluding junction disassembly Relationships: is a type of regulation of cellular component organization [GO:0051128]; regulates tight junction disassembly [GO:1905071] Subtypes: GO:1905074, positive regulation of tight junction disassembly [GO:1905075]